{
  "term_id": "GO:0005635",
  "gene": "UniProtKB:Q96BI1",
  "gene_symbol": "SLC22A18",
  "gene_name": "Solute carrier family 22 member 18",
  "term_label": "nuclear envelope"
}